host cell smooth endoplasmic reticulum membrane [GO:0044171] (CC) Definition: The lipid bilayer surrounding the host cell smooth endoplasmic reticulum. Sources: GOC:jl Also known as: host smooth endoplasmic reticulum membrane Relationships: is a type of GO:0044167; is part of host cell smooth endoplasmic reticulum [GO:0044170]